{
  "gene": "UniProtKB:Q5VZM2",
  "gene_symbol": "RRAGB",
  "term_label": "cellular response to starvation",
  "gene_name": "Ras-related GTP-binding protein B",
  "term_id": "GO:0009267"
}